{
  "gene": "UniProtKB:A6NC51",
  "gene_symbol": "TMEM150B",
  "gene_name": "Modulator of macroautophagy TMEM150B",
  "term_label": "plasma membrane",
  "term_id": "GO:0005886"
}